{
  "gene": "UniProtKB:Q8NGY1",
  "gene_symbol": "OR10Z1",
  "gene_name": "Olfactory receptor 10Z1",
  "term_id": "GO:0004984",
  "term_label": "olfactory receptor activity"
}